{
  "gene": "UniProtKB:Q13651",
  "gene_symbol": "IL10RA",
  "term_label": "interleukin-10 receptor activity",
  "gene_name": "Interleukin-10 receptor subunit alpha",
  "term_id": "GO:0004920"
}